{
  "gene_symbol": "SPRING1",
  "term_label": "Unknown cellular component",
  "term_id": "UNKNOWN:0003",
  "gene": "UniProtKB:Q9H741",
  "gene_name": "SREBP regulating gene protein"
}